{
  "gene_symbol": "NEIL1",
  "term_label": "DNA N-glycosylase activity",
  "gene_name": "Endonuclease 8-like 1",
  "gene": "UniProtKB:Q96FI4",
  "term_id": "GO:0019104"
}